{
  "term_id": "GO:0072659",
  "gene": "UniProtKB:Q86TG1",
  "gene_symbol": "TMEM150A",
  "gene_name": "Transmembrane protein 150A",
  "term_label": "protein localization to plasma membrane"
}